{
  "gene": "UniProtKB:Q5SZD4",
  "gene_symbol": "GLYATL3",
  "term_id": "UNKNOWN:0002",
  "gene_name": "Glycine N-acyltransferase-like protein 3",
  "term_label": "Unknown biological process"
}